negative regulation of serine-type peptidase activity [GO:1902572] (BP) Subtypes: negative regulation of serine-type endopeptidase activity [GO:1900004] Definition: Any process that stops, prevents or reduces the frequency, rate or extent of serine-type peptidase activity. References: PMID:20179351 Sources: GOC:TermGenie, GOC:krc Relationships: is a type of negative regulation of peptidase activity [GO:0010466]; negatively regulates serine-type peptidase activity [GO:0008236] Also known as: down regulation of serine-type peptidase activity, down-regulation of serine-type peptidase activity, downregulation of serine-type peptidase activity, down regulation of serine protease activity, down-regulation of serine protease activity, downregulation of serine protease activity, inhibition of serine protease activity, inhibition of serine-type peptidase activity, negative regulation of serine protease activity